{
  "gene": "UniProtKB:P19623",
  "gene_symbol": "SRM",
  "gene_name": "Spermidine synthase",
  "term_label": "spermidine synthase activity",
  "term_id": "GO:0004766"
}